retrograde axonal transport of mitochondrion [GO:0098958] (biological process) Relationships: is a type of retrograde axonal transport [GO:0008090]; is a type of axonal transport of mitochondrion [GO:0019896] Also known as: retrograde axon transport of mitochondria Sources: GOC:dos Definition: The directed movement of mitochondria along microtubules in axons towards the cell body and away from the presynapse.